{
  "gene": "UniProtKB:O95685",
  "term_label": "protein phosphatase 1 binding",
  "gene_symbol": "PPP1R3D",
  "term_id": "GO:0008157",
  "gene_name": "Protein phosphatase 1 regulatory subunit 3D"
}